{
  "term_id": "GO:0030159",
  "term_label": "signaling receptor complex adaptor activity",
  "gene_name": "Membrane-associated guanylate kinase, WW and PDZ domain-containing protein 2",
  "gene": "UniProtKB:Q86UL8",
  "gene_symbol": "MAGI2"
}